regulation of aggregate size involved in sorocarp development [GO:0031157] (biological process) Definition: Any process that modulates the size of the aggregate formed during sorocarp formation. References: PMID:4338436 Sources: GOC:mah, GOC:mtg_sensu, GOC:pg Also known as: regulation of aggregation during fruiting body biosynthesis, regulation of aggregation during fruiting body formation Relationships: is_a regulation of aggregation involved in sorocarp development [GO:0060176]; is a type of regulation of biological quality [GO:0065008] Subtypes: negative regulation of aggregate size involved in sorocarp development [GO:0031158], positive regulation of aggregate size involved in sorocarp development [GO:0031159]